{
  "term_id": "GO:0003682",
  "gene_name": "Condensin-2 complex subunit H2",
  "gene": "UniProtKB:Q6IBW4",
  "gene_symbol": "NCAPH2",
  "term_label": "chromatin binding"
}